{
  "term_id": "GO:0004222",
  "gene_name": "Matrix metalloproteinase-25",
  "gene": "UniProtKB:Q9NPA2",
  "term_label": "metalloendopeptidase activity",
  "gene_symbol": "MMP25"
}